{
  "term_label": "SNARE binding",
  "gene": "UniProtKB:Q7L8C5",
  "gene_name": "Synaptotagmin-13",
  "term_id": "GO:0000149",
  "gene_symbol": "SYT13"
}